B cell positive selection [GO:0002346] (BP) Sources: GOC:jal Definition: Any process in which B cells are selected to survive based on signaling through the B cell antigen receptor. Also known as: B lymphocyte positive selection, B-cell positive selection, B-lymphocyte positive selection Subtypes: central B cell positive selection [GO:0002348], GO:0002350 Relationships: is a type of B cell selection [GO:0002339]